{
  "gene": "UniProtKB:P59510",
  "term_label": "extracellular matrix",
  "term_id": "GO:0031012",
  "gene_symbol": "ADAMTS20",
  "gene_name": "A disintegrin and metalloproteinase with thrombospondin motifs 20"
}